{
  "gene_symbol": "H2BC10",
  "gene_name": "Histone H2B type 1-C_E_F_G_I",
  "gene": "UniProtKB:P62807",
  "term_id": "GO:0005615",
  "term_label": "extracellular space"
}